{
  "term_label": "cell cortex",
  "gene_symbol": "FAM110C",
  "gene": "UniProtKB:Q1W6H9",
  "gene_name": "Protein FAM110C",
  "term_id": "GO:0005938"
}